{
  "gene_name": "Leiomodin-3",
  "term_id": "GO:0030016",
  "gene": "UniProtKB:Q0VAK6",
  "term_label": "myofibril",
  "gene_symbol": "LMOD3"
}